{
  "term_id": "GO:0005886",
  "gene_symbol": "OR4N4C",
  "gene_name": "Olfactory receptor 4N4C",
  "gene": "UniProtKB:A0A096LPK9",
  "term_label": "plasma membrane"
}